purine deoxyribonucleoside binding [GO:0032547] (molecular function) Definition: Binding to a purine deoxyribonucleoside, a compound consisting of a purine base linked to deoxyribose. Sources: GOC:mah Relationships: is a type of purine nucleoside binding [GO:0001883]; is a type of GO:0032546